{
  "gene": "UniProtKB:A0A1B0GV03",
  "gene_symbol": "GOLGA6L7",
  "term_label": "Unknown molecular function",
  "term_id": "UNKNOWN:0001",
  "gene_name": "Golgin subfamily A member 6-like protein 7"
}